negative regulation of organelle organization [GO:0010639] (biological process) Relationships: is a type of GO:0033043; is a type of negative regulation of cellular component organization [GO:0051129]; negatively regulates GO:0006996 Subtypes: negative regulation of mitochondrial fusion [GO:0010637], GO:0031339, negative regulation of spermatid nuclear differentiation [GO:0045701], negative regulation of cytoskeleton organization [GO:0051494], negative regulation of nuclear division [GO:0051784], negative regulation of vacuole fusion, non-autophagic [GO:0061192], negative regulation of release of cytochrome c from mitochondria [GO:0090201], negative regulation of mitochondrial fission [GO:0090258], negative regulation of lipid droplet fusion [GO:0160078], negative regulation of mitochondrial outer membrane permeabilization involved in apoptotic signaling pathway [GO:1901029], GO:1902116, negative regulation of melanosome organization [GO:1903057], negative regulation of endoplasmic reticulum tubular network organization [GO:1903372], negative regulation of protein insertion into mitochondrial outer membrane [GO:1903637], negative regulation of cristae formation [GO:1903851], negative regulation of secretory granule organization [GO:1904410], GO:1904979, negative regulation of phagosome maturation [GO:1905163], negative regulation of chloroplast fission [GO:1905193], negative regulation of lysosome organization [GO:1905672], negative regulation of postsynaptic density organization [GO:1905875], negative regulation of chromosome organization [GO:2001251] Sources: GOC:dph, GOC:tb Definition: Any process that decreases the frequency, rate or extent of a process involved in the formation, arrangement of constituent parts, or disassembly of an organelle. Also known as: negative regulation of organelle organisation, negative regulation of organelle organization and biogenesis